{
  "term_id": "UNKNOWN:0002",
  "gene": "UniProtKB:Q8IUS5",
  "gene_name": "Epoxide hydrolase 4",
  "term_label": "Unknown biological process",
  "gene_symbol": "EPHX4"
}